D-alanine [D-alanyl carrier protein] ligase activity [GO:0047473] (molecular function) Definition: Catalysis of the ATP-dependent activation of D-alanine and its transfer as a thiol ester to the phosphopantheinyl prosthetic group of a D-alanyl carrier protein, according to the reaction: ATP + D-alanine + a [D-alaninyl carrier protein] = a D-alanyl-[D-alanyl carrier protein] + AMP + diphosphate. Relationships: is a type of GO:0016878 Sources: GOC:pg Also known as: D-alanine-poly(phosphoribitol) ligase activity, D-alanine:poly(phosphoribitol) ligase (AMP-forming), D-alanine-D-alanyl carrier protein ligase activity, D-alanine-activating enzyme activity